hydrocarbon biosynthetic process [GO:0120251] (biological process) Definition: The chemical reactions and pathways resulting in the formation of a hydrocarbon, a compound consisting of carbon and hydrogen only. Also known as: hydrocarbon anabolism, hydrocarbon biosynthesis, hydrocarbon formation, hydrocarbon synthesis Subtypes: cuticle hydrocarbon biosynthetic process [GO:0006723], alkane biosynthetic process [GO:0043447], alkyne biosynthetic process [GO:0043453], terpene biosynthetic process [GO:0046246], toluene biosynthetic process [GO:0046252], olefin biosynthetic process [GO:1900674], benzene biosynthetic process [GO:1900997] Sources: GOC:krc, Wikipedia:Hydrocarbon Relationships: is a type of biosynthetic process [GO:0009058]; is a type of hydrocarbon metabolic process [GO:0120252]